{
  "gene_symbol": "MAFF",
  "term_id": "GO:0006357",
  "gene_name": "Transcription factor MafF",
  "gene": "UniProtKB:Q9ULX9",
  "term_label": "regulation of transcription by RNA polymerase II"
}